presynaptic actin cytoskeleton [GO:0099143] (cellular component) Sources: GOC:dos Definition: The actin cytoskeleton that is part of a presynapse. Relationships: is a type of actin cytoskeleton [GO:0015629]; is a type of presynaptic cytoskeleton [GO:0099569]